melanization of appressorium wall [GO:0075043] (biological process) Definition: The process in which melanin is produced in the appressorium of the symbiont. Melanization of the appressorium increases turgor pressure in the appressorium. Also known as: melanization of appressorium to maintain turgor pressure, maintenance of turgor in appressorium by melanization Relationships: is a type of pigment accumulation [GO:0043476]; is part of appressorium maturation [GO:0075035]; has part melanin biosynthetic process [GO:0042438] References: PMID:28165657 Sources: GOC:pamgo_curators, Wikipedia:Appressorium